4-oxalmesaconate hydratase activity [GO:0047584] (molecular function) Also known as: 2-hydroxy-4-oxobutane-1,2,4-tricarboxylate 2,3-hydro-lyase [(E)-4-oxobut-1-ene-1,2,4-tricarboxylate-forming], 2-hydroxy-4-oxobutane-1,2,4-tricarboxylate 2,3-hydro-lyase activity, 4-carboxy-2-oxobutane-1,2,4-tricarboxylate 2,3-hydro-lyase activity, 4-carboxy-2-oxohexenedioate hydratase activity, gamma-oxalmesaconate hydratase activity, oxalmesaconate hydratase activity Relationships: is a type of hydro-lyase activity [GO:0016836] Sources: EC:4.2.1.83, RHEA:17401 Definition: Catalysis of the reaction: 2-hydroxy-4-oxobutane-1,2,4-tricarboxylate = (1E)-4-oxobut-1-ene-1,2,4-tricarboxylate + H2O.